{
  "term_label": "RNA polymerase II cis-regulatory region sequence-specific DNA binding",
  "gene_name": "Hepatocyte nuclear factor 6",
  "gene": "UniProtKB:Q9UBC0",
  "gene_symbol": "ONECUT1",
  "term_id": "GO:0000978"
}